negative regulation of iron ion transmembrane transport [GO:0034760] (biological process) Relationships: is a type of GO:0034757; is a type of regulation of iron ion transmembrane transport [GO:0034759]; is a type of negative regulation of cation transmembrane transport [GO:1904063]; negatively regulates iron ion transmembrane transport [GO:0034755] Sources: GOC:mah Also known as: down regulation of transmembrane iron ion transport, down-regulation of transmembrane iron ion transport, downregulation of transmembrane iron ion transport, negative regulation of iron ion membrane transport, negative regulation of transmembrane iron ion transport, negative regulation of transmembrane iron transport, inhibition of transmembrane iron ion transport Definition: Any process that stops, prevents, or reduces the frequency, rate or extent of the directed movement of iron ions from one side of a membrane to the other by means of some agent such as a transporter or pore. Subtypes: GO:1904039, GO:1904439